{
  "gene": "UniProtKB:Q8WXS4",
  "term_label": "Unknown biological process",
  "gene_symbol": "TMEM37",
  "term_id": "UNKNOWN:0002",
  "gene_name": "Voltage-dependent calcium channel gamma-like subunit"
}